{
  "gene_symbol": "CLPP",
  "gene_name": "ATP-dependent Clp protease proteolytic subunit, mitochondrial",
  "gene": "UniProtKB:Q16740",
  "term_id": "GO:0009368",
  "term_label": "endopeptidase Clp complex"
}